response to UV [GO:0009411] (biological process) Sources: GOC:hb Relationships: is a type of response to light stimulus [GO:0009416] Also known as: response to UV light stimulus, response to UV radiation stimulus, response to ultraviolet light stimulus, response to ultraviolet radiation stimulus Definition: Any process that results in a change in state or activity of a cell or an organism (in terms of movement, secretion, enzyme production, gene expression, etc.) as a result of an ultraviolet radiation (UV light) stimulus. Ultraviolet radiation is electromagnetic radiation with a wavelength in the range of 10 to 380 nanometers. Subtypes: detection of UV [GO:0009589], UV protection [GO:0009650], response to UV-B [GO:0010224], response to UV-C [GO:0010225], cellular response to UV [GO:0034644], pigment accumulation in response to UV light [GO:0043478], response to UV-A [GO:0070141]